{
  "term_label": "endoplasmic reticulum membrane",
  "gene": "UniProtKB:A4D0T7",
  "gene_symbol": "SMIM30",
  "term_id": "GO:0005789",
  "gene_name": "Small integral membrane protein 30"
}